{
  "gene_name": "Homeobox protein CDX-2",
  "term_id": "GO:0003700",
  "term_label": "DNA-binding transcription factor activity",
  "gene": "UniProtKB:Q99626",
  "gene_symbol": "CDX2"
}